acetylcholine-gated channel complex [GO:0005892] (cellular component) References: PMID:12381728, PMID:15579462 Sources: GOC:bf, GOC:mah Definition: A homo- or hetero-pentameric protein complex that forms a transmembrane channel through which ions may pass in response to acetylcholine binding. Also known as: nicotinic acetylcholine receptor, nicotinic acetylcholine-gated receptor-channel complex Relationships: is a type of monoatomic ion channel complex [GO:0034702]; is a type of GO:0098802